{
  "gene_symbol": "LRRK1",
  "gene_name": "Leucine-rich repeat serine_threonine-protein kinase 1",
  "gene": "UniProtKB:Q38SD2",
  "term_label": "Unknown biological process",
  "term_id": "UNKNOWN:0002"
}